{
  "gene_symbol": "PHB1",
  "term_label": "mitochondrion organization",
  "gene": "UniProtKB:P35232",
  "term_id": "GO:0007005",
  "gene_name": "Prohibitin 1"
}